left ventral basal body [GO:1902675] (cellular component) References: PMID:16607022, PMID:5961344 Sources: GOC:TermGenie, GOC:giardia, GO_REF:0000064, ISBN:9780124260207 Note: Note that we deem cilium and microtubule-based flagellum to be equivalent. Also note that, due to the asymmetric nature of the Giardia trophozoite, this term is defined spatially as the trophozoite is viewed from the dorsal side, with the two nuclei dorsal to the ventral disc, and the ventral disc toward the anterior. Relationships: is a type of ciliary basal body [GO:0036064]; is part of left ventral flagellum [GO:0097558] Definition: Any ciliary basal body that is part of a left ventral flagellum found in Giardia species (trophozoite stage). Also known as: cilial basal body of left ventral cilium, cilial basal body of left ventral flagellum, ciliary basal body of left ventral cilium, ciliary basal body of left ventral flagellum, cilium basal body of left ventral cilium, cilium basal body of left ventral flagellum, left ventral flagellum ciliary basal body, microtubule basal body of left ventral cilium, microtubule basal body of left ventral flagellum